{
  "term_label": "spindle assembly",
  "gene": "UniProtKB:Q96CS2",
  "gene_symbol": "HAUS1",
  "term_id": "GO:0051225",
  "gene_name": "HAUS augmin-like complex subunit 1"
}